{
  "gene_symbol": "SLC22A20P",
  "term_id": "GO:0015711",
  "term_label": "organic anion transport",
  "gene_name": "Solute carrier family 22 member 20",
  "gene": "UniProtKB:A6NK97"
}